regulation of cellulose biosynthetic process [GO:2001006] (biological process) Subtypes: GO:2001007, positive regulation of cellulose biosynthetic process [GO:2001008], regulation of plant-type cell wall cellulose biosynthetic process [GO:2001009] Definition: Any process that modulates the frequency, rate or extent of cellulose biosynthetic process. Sources: GOC:mengo_curators Relationships: is a type of GO:0032951; regulates GO:0030244 Also known as: regulation of cellulose anabolism, regulation of cellulose biosynthesis, regulation of cellulose formation, regulation of cellulose synthesis